{
  "gene_name": "Olfactory receptor 2H2",
  "gene": "UniProtKB:O95918",
  "term_label": "plasma membrane",
  "gene_symbol": "OR2H2",
  "term_id": "GO:0005886"
}